{
  "term_label": "cilium movement involved in cell motility",
  "gene_name": "Dynein axonemal heavy chain 6",
  "gene": "UniProtKB:Q9C0G6",
  "gene_symbol": "DNAH6",
  "term_id": "GO:0060294"
}